{
  "gene_name": "Hepatocyte growth factor activator",
  "term_id": "GO:0007596",
  "term_label": "blood coagulation",
  "gene": "UniProtKB:Q04756",
  "gene_symbol": "HGFAC"
}